{
  "term_id": "UNKNOWN:0001",
  "gene_name": "Small ribosomal subunit protein bS21m",
  "term_label": "Unknown molecular function",
  "gene_symbol": "MRPS21",
  "gene": "UniProtKB:P82921"
}